{
  "gene": "UniProtKB:Q5TDH0",
  "gene_symbol": "DDI2",
  "term_id": "GO:0031647",
  "term_label": "regulation of protein stability",
  "gene_name": "Protein DDI1 homolog 2"
}